{
  "gene_name": "Putative translationally-controlled tumor protein-like protein TPT1P8",
  "gene_symbol": "TPT1P8",
  "gene": "UniProtKB:Q9HAU6",
  "term_label": "Unknown biological process",
  "term_id": "UNKNOWN:0002"
}